{
  "term_label": "C-C chemokine receptor activity",
  "term_id": "GO:0016493",
  "gene_symbol": "GPR75",
  "gene": "UniProtKB:O95800",
  "gene_name": "Probable G-protein coupled receptor 75"
}